succinylornithine transaminase activity [GO:0043825] (molecular function) Also known as: succinylornithine aminotransferase activity, N2-succinyl-L-ornithine:2-oxoglutarate 5-aminotransferase activity, N2-succinylornithine 5-aminotransferase activity, succinyl ornithine transaminase activity, 2-N-succinyl-L-ornithine:2-oxoglutarate 5-aminotransferase activity, AstC, N(2)-succinylornithine 5-aminotransferase activity, SOAT, succinyl-ornithine transaminase activity Relationships: is a type of transaminase activity [GO:0008483] Definition: Catalysis of the reaction: 2-oxoglutarate + N(2)-succinyl-L-ornithine = N-succinyl-L-glutamate 5-semialdehyde + L-glutamate. Sources: EC:2.6.1.81, RHEA:16953